{
  "gene_symbol": "TXNRD3",
  "gene": "UniProtKB:Q86VQ6",
  "term_label": "mitochondrion",
  "gene_name": "Thioredoxin reductase 3",
  "term_id": "GO:0005739"
}